{
  "gene_name": "Kinesin-like protein KIF2A",
  "term_label": "kinesin complex",
  "gene": "UniProtKB:O00139",
  "gene_symbol": "KIF2A",
  "term_id": "GO:0005871"
}